spicule insertion [GO:0034609] (biological process) References: PMID:18050467 Relationships: is a type of male mating behavior [GO:0060179] Definition: Insertion of the male copulatory spicules into the hermaphrodite. Spicule insertion behavior initiates when the male cloaca contacts the vulva. During most mating encounters, the spicule tips will prod the vulva continuously until they partially penetrate, which then causes the protractors to contract completely so that the spicules extend through the vulva.